{
  "term_label": "respiratory chain complex",
  "gene_symbol": "COX7A2P2",
  "term_id": "GO:0098803",
  "gene": "UniProtKB:O60397",
  "gene_name": "Putative cytochrome c oxidase subunit 7A3, mitochondrial"
}